positive regulation of violaceol II biosynthetic process [GO:1900718] (biological process) Sources: GOC:TermGenie, GOC:di Definition: Any process that activates or increases the frequency, rate or extent of violaceol II biosynthetic process. Relationships: is a type of GO:1900378; is a type of regulation of violaceol II biosynthetic process [GO:1900716]; positively regulates violaceol II biosynthetic process [GO:1900593] Also known as: activation of violaceol II anabolism, activation of violaceol II biosynthesis, activation of violaceol II formation, activation of violaceol II synthesis, positive regulation of violaceol II anabolism, positive regulation of violaceol II biosynthesis, positive regulation of violaceol II formation, positive regulation of violaceol II synthesis, up regulation of violaceol II anabolism, up regulation of violaceol II biosynthesis, up regulation of violaceol II biosynthetic process, up regulation of violaceol II formation, up regulation of violaceol II synthesis, up-regulation of violaceol II anabolism, up-regulation of violaceol II biosynthesis, up-regulation of violaceol II biosynthetic process, up-regulation of violaceol II formation, up-regulation of violaceol II synthesis, upregulation of violaceol II anabolism, upregulation of violaceol II biosynthesis, upregulation of violaceol II biosynthetic process, upregulation of violaceol II formation, upregulation of violaceol II synthesis, activation of violaceol II biosynthetic process